spermatid cytoplasm removal during spermiation of flagellated sperm [GO:0160087] (BP) References: PMID:21866274, PMID:23087837 Relationships: is a type of developmental process involved in reproduction [GO:0003006]; is part of spermatogenesis [GO:0007283] Definition: The process of removing the majority of the cytoplasm and organelles from a spermatid as it develops into a mature flagellated sperm cell.